{
  "gene_symbol": "TRIM2",
  "term_id": "GO:0000209",
  "gene": "UniProtKB:Q9C040",
  "gene_name": "Tripartite motif-containing protein 2",
  "term_label": "protein polyubiquitination"
}